{
  "gene_symbol": "SLC20A1",
  "gene_name": "Sodium-dependent phosphate transporter 1",
  "gene": "UniProtKB:Q8WUM9",
  "term_label": "Unknown cellular component",
  "term_id": "UNKNOWN:0003"
}